{
  "term_label": "protein transporter activity",
  "gene_symbol": "TIMM9",
  "gene_name": "Mitochondrial import inner membrane translocase subunit Tim9",
  "gene": "UniProtKB:Q9Y5J7",
  "term_id": "GO:0140318"
}